{
  "gene": "UniProtKB:P20671",
  "term_id": "GO:0030527",
  "gene_symbol": "H2AC7",
  "term_label": "structural constituent of chromatin",
  "gene_name": "Histone H2A type 1-D"
}